{
  "term_label": "plasma membrane",
  "term_id": "GO:0005886",
  "gene_name": "Adhesion G protein-coupled receptor E1",
  "gene": "UniProtKB:Q14246",
  "gene_symbol": "ADGRE1"
}